{
  "term_label": "Unknown molecular function",
  "gene": "UniProtKB:Q1ZYL8",
  "term_id": "UNKNOWN:0001",
  "gene_name": "Izumo sperm-egg fusion protein 4",
  "gene_symbol": "IZUMO4"
}